{
  "gene_symbol": "CCNI2",
  "term_id": "GO:0005737",
  "term_label": "cytoplasm",
  "gene_name": "Cyclin-I2",
  "gene": "UniProtKB:Q6ZMN8"
}